{
  "term_label": "regulation of transcription by RNA polymerase II",
  "gene": "UniProtKB:O75461",
  "gene_name": "Transcription factor E2F6",
  "gene_symbol": "E2F6",
  "term_id": "GO:0006357"
}